{
  "gene": "UniProtKB:O60921",
  "term_label": "nucleotide-excision repair",
  "term_id": "GO:0006289",
  "gene_name": "Checkpoint protein HUS1",
  "gene_symbol": "HUS1"
}